{
  "term_label": "olfactory receptor activity",
  "term_id": "GO:0004984",
  "gene_symbol": "OR1F1",
  "gene_name": "Olfactory receptor 1F1",
  "gene": "UniProtKB:O43749"
}